5-amino-6-(5-phosphoribitylamino)uracil phosphatase activity [GO:0043726] (MF) Definition: Catalysis of the reaction: 5-amino-6-(5-phospho-D-ribitylamino)uracil + H2O = 5-amino-6-(D-ribitylamino)uracil + phosphate. Also known as: pyrimidine phosphatase activity Relationships: is a type of phosphatase activity [GO:0016791] Sources: GOC:jl